regulation of regulatory ncRNA processing [GO:0070920] (biological process) Relationships: is a type of regulation of gene silencing by regulatory ncRNA [GO:0060966]; is a type of GO:0080090; regulates regulatory ncRNA processing [GO:0070918] Also known as: regulation of gene silencing by RNA, production of guide RNA, regulation of gene silencing by RNA, production of small RNA, regulation of production of small RNA involved in gene silencing by RNA Sources: GOC:mah Subtypes: GO:0070921, GO:1903798 Definition: Any process that modulates the frequency, rate or extent of regulatory non-coding RNA processing.